{
  "gene": "UniProtKB:Q9UNE7",
  "term_id": "GO:0071218",
  "gene_symbol": "STUB1",
  "gene_name": "E3 ubiquitin-protein ligase CHIP",
  "term_label": "cellular response to misfolded protein"
}